negative regulation of zinc ion transport [GO:0071582] (biological process) Definition: Any process that stops, prevents, or reduces the frequency, rate or extent of the directed movement of zinc ions (Zn2+) into, out of or within a cell, or between cells, by means of some agent such as a transporter or pore. Sources: GOC:BHF, GOC:mah Subtypes: negative regulation of zinc ion transmembrane transport [GO:0071583] Relationships: is a type of negative regulation of monoatomic ion transport [GO:0043271]; is_a regulation of zinc ion transport [GO:0071579]; negatively regulates zinc ion transport [GO:0006829]